{
  "gene_symbol": "FOXF1",
  "term_id": "GO:0000978",
  "term_label": "RNA polymerase II cis-regulatory region sequence-specific DNA binding",
  "gene": "UniProtKB:Q12946",
  "gene_name": "Forkhead box protein F1"
}